chloroplast ribosome [GO:0043253] (cellular component) Sources: GOC:ecd Relationships: is a type of plastid ribosome [GO:0009547]; is part of chloroplast stroma [GO:0009570] Definition: A ribosome contained within a chloroplast.